{
  "term_label": "nucleus",
  "gene": "UniProtKB:Q15847",
  "term_id": "GO:0005634",
  "gene_name": "Adipogenesis regulatory factor",
  "gene_symbol": "ADIRF"
}